{
  "term_label": "ephrin receptor signaling pathway",
  "gene_symbol": "EPHA10",
  "gene": "UniProtKB:Q5JZY3",
  "term_id": "GO:0048013",
  "gene_name": "Ephrin type-A receptor 10"
}